{
  "gene_symbol": "FTH1P19",
  "gene_name": "Putative ferritin heavy polypeptide-like 19",
  "term_id": "GO:0005737",
  "term_label": "cytoplasm",
  "gene": "UniProtKB:P0C7X4"
}